signaling receptor activator activity [GO:0030546] (molecular function) Sources: GOC:ceb Subtypes: transmembrane receptor protein tyrosine kinase activator activity [GO:0030297], acetylcholine receptor activator activity [GO:0030549], receptor ligand activity [GO:0048018] Relationships: is_a signaling receptor regulator activity [GO:0030545]; is a type of molecular function activator activity [GO:0140677]; positively regulates signaling receptor activity [GO:0038023] Definition: The function of interacting (directly or indirectly) with receptors such that the proportion of receptors in the active form is increased. Also known as: receptor activator activity, signalling receptor activator activity